{
  "gene": "UniProtKB:Q8WUX9",
  "term_label": "nuclear envelope",
  "gene_name": "Charged multivesicular body protein 7",
  "term_id": "GO:0005635",
  "gene_symbol": "CHMP7"
}